lactose metabolic process [GO:0005988] (biological process) Relationships: is a type of disaccharide metabolic process [GO:0005984] Subtypes: GO:0005989, lactose catabolic process [GO:0005990] Sources: GOC:go_curators Also known as: lactose metabolism Definition: The chemical reactions and pathways involving lactose, the disaccharide galactopyranosyl-glucose.